{
  "term_id": "GO:0019773",
  "gene_name": "Proteasome subunit alpha type-1",
  "gene": "UniProtKB:P25786",
  "term_label": "proteasome core complex, alpha-subunit complex",
  "gene_symbol": "PSMA1"
}